{
  "term_id": "GO:0016485",
  "term_label": "protein processing",
  "gene": "UniProtKB:P16870",
  "gene_name": "Carboxypeptidase E",
  "gene_symbol": "CPE"
}